{
  "gene": "UniProtKB:Q9NX36",
  "term_id": "UNKNOWN:0003",
  "term_label": "Unknown cellular component",
  "gene_name": "DnaJ homolog subfamily C member 28",
  "gene_symbol": "DNAJC28"
}